{
  "gene_symbol": "BVES",
  "gene_name": "Blood vessel epicardial substance",
  "term_id": "GO:0007519",
  "gene": "UniProtKB:Q8NE79",
  "term_label": "skeletal muscle tissue development"
}